{
  "gene_name": "Small integral membrane protein 15",
  "term_label": "Unknown biological process",
  "gene_symbol": "SMIM15",
  "gene": "UniProtKB:Q7Z3B0",
  "term_id": "UNKNOWN:0002"
}